embryonic medial fin morphogenesis [GO:0035122] (biological process) Also known as: embryonic unpaired fin morphogenesis Sources: GOC:dgh Relationships: is a type of embryonic appendage morphogenesis [GO:0035113]; is_a medial fin morphogenesis [GO:0035141] Subtypes: embryonic dorsal fin morphogenesis [GO:0035123], embryonic caudal fin morphogenesis [GO:0035124], embryonic anal fin morphogenesis [GO:0035125] Definition: The process, occurring in the embryo, by which the anatomical structures of the medial fin are generated and organized. Medial fins are unpaired fins of fish, usually located dorsomedially or ventromedially and primarily used for stability while swimming.